{
  "gene": "UniProtKB:O43291",
  "term_id": "UNKNOWN:0003",
  "term_label": "Unknown cellular component",
  "gene_name": "Kunitz-type protease inhibitor 2",
  "gene_symbol": "SPINT2"
}